protoporphyrinogen IX biosynthetic process from glycine [GO:0019352] (biological process) Definition: The chemical reactions and pathways resulting in the formation of protoporphyrinogen IX from other compounds, including glycine. Relationships: is_a GO:0006544; is a type of GO:0006782 Sources: GOC:go_curators Also known as: protoporphyrinogen IX anabolism from glycine, protoporphyrinogen IX formation from glycine, protoporphyrinogen IX synthesis from glycine